23S rRNA pseudouridine(2604) synthase activity [GO:0160138] (molecular function) Definition: Catalysis of the reaction: uridine(2604) in 23S rRNA = pseudouridine(2604) in 23S rRNA. Sources: EC:5.4.99.21, RHEA:38875 Relationships: is a type of rRNA pseudouridine synthase activity [GO:0120159]